{
  "gene_symbol": "WDR87",
  "term_id": "UNKNOWN:0003",
  "gene_name": "WD repeat-containing protein 87",
  "term_label": "Unknown cellular component",
  "gene": "UniProtKB:Q6ZQQ6"
}